{
  "gene": "UniProtKB:Q99732",
  "gene_symbol": "LITAF",
  "term_label": "cytoplasmic side of lysosomal membrane",
  "term_id": "GO:0098574",
  "gene_name": "Lipopolysaccharide-induced tumor necrosis factor-alpha factor"
}